{
  "gene_name": "Cardiomyopathy-associated protein 5",
  "term_id": "UNKNOWN:0001",
  "term_label": "Unknown molecular function",
  "gene": "UniProtKB:Q8N3K9",
  "gene_symbol": "CMYA5"
}